salivary gland boundary specification [GO:0007432] (BP) Regulation: regulated by regulation of salivary gland boundary specification [GO:0045704]; negatively regulated by negative regulation of salivary gland boundary specification [GO:0045705]; positively regulated by GO:0045706 References: PMID:11598957 Relationships: is a type of GO:0010160; is part of salivary gland development [GO:0007431] Also known as: salivary gland determination Subtypes: larval salivary gland boundary specification [GO:0007433], GO:0007434 Definition: Determination of where the salivary gland forms, the total number of salivary gland cells and how many cells are allocated to each of the specialised cell types within the salivary gland.